cysteine-S-conjugate beta-lyase activity [GO:0047804] (molecular function) Definition: Catalysis of the reaction: S-substituted L-cysteine + H2O = a thiol + NH4+ + pyruvate. Relationships: is a type of carbon-sulfur lyase activity [GO:0016846] Also known as: cysteine-S-conjugate b-lyase activity, L-cysteine-S-conjugate thiol-lyase (deaminating) activity, L-cysteine-S-conjugate thiol-lyase (deaminating; pyruvate-forming), S-alkylcysteine lyase activity, alkylcysteine lyase activity, cystathionine beta-lyase activity, cysteine conjugate beta-lyase activity, glutamine transaminase K/cysteine conjugate beta-lyase activity Sources: RHEA:18121